{
  "term_label": "cytoplasm",
  "gene_name": "Coiled-coil domain-containing protein 50",
  "term_id": "GO:0005737",
  "gene": "UniProtKB:Q8IVM0",
  "gene_symbol": "CCDC50"
}